plasmodesmatal desmotubule [GO:0009510] (cellular component) Relationships: is a type of GO:0110165; is part of GO:0005783; is part of plasma membrane [GO:0005886]; is part of plasmodesma [GO:0009506] References: PMID:29880547 Also known as: desmotubule central rod Definition: A tightly wound cylinder of membrane that is located within the plasmodesmal pore and runs the length of the plasmodesma. The desmotubule likely provides a rigid stability to plasmodesmata and confers a fixed diameter and pore size to the plasmodesmal canal, and is linked to the endoplasmic reticulum in each of the adjacent cell.